{
  "term_id": "GO:0006915",
  "term_label": "apoptotic process",
  "gene": "UniProtKB:Q9BRP1",
  "gene_name": "Programmed cell death protein 2-like",
  "gene_symbol": "PDCD2L"
}